vestibulocochlear nerve maturation [GO:0021647] (biological process) Also known as: CN VIII maturation, auditory nerve maturation Relationships: is a type of cranial nerve maturation [GO:0021605]; is part of vestibulocochlear nerve development [GO:0021562] Definition: A developmental process, independent of morphogenetic (shape) change, that is required for the vestibulocochlear nerve to attain its fully functional state. This sensory nerve innervates the membranous labyrinth of the inner ear. The vestibular branch innervates the vestibular apparatus that senses head position changes relative to gravity. The auditory branch innervates the cochlear duct, which is connected to the three bony ossicles which transduce sound waves into fluid movement in the cochlea. Sources: GOC:cls, GOC:dgh, GOC:dph, GOC:jid, GO_REF:0000021